Pup conjugating enzyme activity [GO:0061655] (MF) Also known as: E2 Relationships: is_a GO:0061650; is a type of Pup transferase activity [GO:0072496] Sources: GOC:dph Definition: Isoenergetic transfer of Pup from one protein to another via the reaction X-Pup + Y = Y-Pup + X, where both the X-Pup and Y-Pup linkages are thioester bonds between the C-terminal amino acid of Pup and a sulfhydryl side group of a cysteine residue.